zymogen activation [GO:0031638] (biological process) Definition: The proteolytic processing of an inactive enzyme to an active form. Sources: GOC:hjd Also known as: zymogen activation by proteolytic cleavage Subtypes: plasminogen activation [GO:0031639], trypsinogen activation [GO:0032023] Relationships: is a type of protein processing [GO:0016485]